{
  "gene_symbol": "PAPPA-AS1",
  "term_label": "Unknown molecular function",
  "gene": "UniProtKB:Q5QFB9",
  "term_id": "UNKNOWN:0001",
  "gene_name": "Protein PAPPAS"
}